negative regulation of transport [GO:0051051] (biological process) Relationships: is a type of negative regulation of biological process [GO:0048519]; is a type of GO:0051049; negatively regulates GO:0006810 Subtypes: negative regulation of vesicle fusion [GO:0031339], negative regulation of nucleobase-containing compound transport [GO:0032240], negative regulation of lipid transport [GO:0032369], negative regulation of intracellular transport [GO:0032387], GO:0032410, negative regulation of organic acid transport [GO:0032891], negative regulation of transmembrane transport [GO:0034763], negative regulation of SNARE complex disassembly [GO:0035541], negative regulation of monoatomic ion transport [GO:0043271], negative regulation of endocytosis [GO:0045806], GO:0051048, GO:0051224, negative regulation of neurotransmitter transport [GO:0051589], negative regulation of norepinephrine uptake [GO:0051622], negative regulation of epinephrine uptake [GO:0051627], GO:0051953, GO:0106021, negative regulation of transport across blood-brain barrier [GO:0150202], negative regulation of cellotriose transport [GO:1900286], negative regulation of galactotriose transport [GO:1900292], negative regulation of heptasaccharide transport [GO:1900295], GO:1900298, negative regulation of laminaritriose transport [GO:1900304], negative regulation of maltotetraose transport [GO:1900322], negative regulation of maltotriulose transport [GO:1900325], GO:1900328, GO:1900358, negative regulation of pentasaccharide transport [GO:1900361], negative regulation of peptide antigen transport [GO:1901040], negative regulation of maltose transport [GO:1902344], negative regulation of synaptic vesicle transport [GO:1902804], negative regulation of melanosome transport [GO:1902909], negative regulation of synaptic vesicle recycling [GO:1903422], GO:1904299, negative regulation of intralumenal vesicle formation [GO:1905366], GO:2000119, GO:2000808, GO:2000877, negative regulation of renal water transport [GO:2001152] Sources: GOC:ai Also known as: down regulation of transport, down-regulation of transport, downregulation of transport, inhibition of transport Definition: Any process that stops, prevents, or reduces the frequency, rate or extent of the directed movement of substances (such as macromolecules, small molecules, ions) into, out of or within a cell, or between cells, by means of some agent such as a transporter or pore.